Schaffer collateral - CA1 synapse [GO:0098685] (cellular component) Relationships: is_a synapse [GO:0045202] References: PMID:16399689 Definition: A synapse between the Schaffer collateral axon of a CA3 pyramidal cell and a CA1 pyramidal cell.